{
  "gene_name": "Renal cancer differentiation gene 1 protein",
  "term_label": "Unknown molecular function",
  "term_id": "UNKNOWN:0001",
  "gene": "UniProtKB:Q504U0",
  "gene_symbol": "C4orf46"
}